{
  "term_id": "UNKNOWN:0001",
  "term_label": "Unknown molecular function",
  "gene_symbol": "ERMARD",
  "gene_name": "Endoplasmic reticulum membrane-associated RNA degradation protein",
  "gene": "UniProtKB:Q5T6L9"
}